{
  "term_label": "Unknown molecular function",
  "gene": "UniProtKB:Q8N766",
  "gene_name": "ER membrane protein complex subunit 1",
  "gene_symbol": "EMC1",
  "term_id": "UNKNOWN:0001"
}